{
  "gene_symbol": "ZNF892",
  "term_label": "regulation of transcription by RNA polymerase II",
  "gene_name": "Zinc finger protein 892",
  "gene": "UniProtKB:A0A087WUV0",
  "term_id": "GO:0006357"
}